{
  "gene_name": "Activator of basal transcription 1",
  "term_id": "GO:0000472",
  "term_label": "endonucleolytic cleavage to generate mature 5'-end of SSU-rRNA from (SSU-rRNA, 5.8S rRNA, LSU-rRNA)",
  "gene_symbol": "ABT1",
  "gene": "UniProtKB:Q9ULW3"
}